rhombomere 1 morphogenesis [GO:0021651] (biological process) Relationships: is_a rhombomere morphogenesis [GO:0021593]; is part of rhombomere 1 development [GO:0021567] Sources: GOC:cls, GOC:curators, GOC:dgh, GOC:dph, GOC:jid Definition: The process in which the anatomical structure of rhombomere 1 is generated and organized. Rhombomeres are transverse segments of the developing rhombencephalon. Rhombomeres are lineage restricted, express different genes from one another, and adopt different developmental fates. Rhombomeres are numbered in an anterior to posterior order.